positive regulation of vitamin D receptor signaling pathway [GO:0070564] (biological process) Sources: GOC:BHF, GOC:mah Relationships: is a type of regulation of vitamin D receptor signaling pathway [GO:0070562]; is a type of positive regulation of intracellular signal transduction [GO:1902533]; positively regulates vitamin D receptor signaling pathway [GO:0070561] Definition: Any process that activates or increases the frequency, rate or extent of vitamin D receptor signaling pathway activity. Also known as: positive regulation of VDR signaling pathway, positive regulation of vitamin D receptor signalling pathway, up regulation of vitamin D receptor signaling pathway, up-regulation of vitamin D receptor signaling pathway, upregulation of vitamin D receptor signaling pathway, activation of vitamin D receptor signaling pathway, stimulation of vitamin D receptor signaling pathway